{
  "term_id": "GO:0051180",
  "gene": "UniProtKB:P43652",
  "gene_symbol": "AFM",
  "term_label": "vitamin transport",
  "gene_name": "Afamin"
}